protein localization to non-growing cell tip [GO:1902487] (biological process) Relationships: is a type of GO:1990151 References: PMID:21652630, PMID:23041194 Sources: GOC:TermGenie Definition: A process in which a protein is transported to, or maintained in, a location within a non-growing cell tip. Also known as: protein localisation in non-growing cell tip, protein localisation to non-growing cell tip, protein localization in non-growing cell tip Regulation: regulated by GO:0062107; negatively regulated by GO:0062108